glycopeptide catabolic process [GO:0009050] (biological process) Relationships: is a type of amide metabolic process [GO:0043603]; is a type of GO:1901136 Sources: GOC:go_curators, ISBN:0198506732 Also known as: glycopeptide breakdown, glycopeptide catabolism, glycopeptide degradation Definition: The chemical reactions and pathways resulting in the breakdown of glycopeptides, a compound in which carbohydrate is covalently attached to an oligopeptide composed of residues of L and/or D-amino acids. The term usually denotes a product of proteolytic degradation of a glycoprotein but includes glycated peptide.